{
  "gene_name": "Putative activator of 90 kDa heat shock protein ATPase homolog 2",
  "term_id": "GO:0005829",
  "gene_symbol": "AHSA2P",
  "term_label": "cytosol",
  "gene": "UniProtKB:Q719I0"
}